{
  "gene": "UniProtKB:Q0JRZ9",
  "gene_name": "F-BAR domain only protein 2",
  "gene_symbol": "FCHO2",
  "term_id": "GO:0030136",
  "term_label": "clathrin-coated vesicle"
}